{
  "gene_symbol": "DHH",
  "gene_name": "Desert hedgehog protein",
  "term_label": "patched binding",
  "term_id": "GO:0005113",
  "gene": "UniProtKB:O43323"
}